{
  "term_id": "GO:0002040",
  "gene_symbol": "VEGFA",
  "gene_name": "Vascular endothelial growth factor A, long form",
  "term_label": "sprouting angiogenesis",
  "gene": "UniProtKB:P15692"
}